{
  "gene": "UniProtKB:P08253",
  "term_label": "response to hypoxia",
  "gene_symbol": "MMP2",
  "gene_name": "72 kDa type IV collagenase",
  "term_id": "GO:0001666"
}